regulation of mammary gland involution [GO:1903519] (biological process) Subtypes: negative regulation of mammary gland involution [GO:1903520], positive regulation of mammary gland involution [GO:1903521] Definition: Any process that modulates the frequency, rate or extent of mammary gland involution. Relationships: is a type of regulation of tissue remodeling [GO:0034103]; RO_0002211 mammary gland involution [GO:0060056] References: PMID:23164222 Sources: GOC:TermGenie, GOC:dph, GO_REF:0000058